{
  "gene_name": "Aldehyde dehydrogenase family 3 member A2",
  "term_label": "3-chloroallyl aldehyde dehydrogenase activity",
  "term_id": "GO:0004028",
  "gene_symbol": "ALDH3A2",
  "gene": "UniProtKB:P51648"
}